phosphonopyruvate hydrolase activity [GO:0033978] (molecular function) Relationships: is a type of GO:0016827 Definition: Catalysis of the reaction: 3-phosphonopyruvate + H2O = H+ + phosphate + pyruvate. Also known as: PPH Sources: RHEA:16673